D-threo-aldose 1-dehydrogenase activity [GO:0047834] (molecular function) Also known as: (2S,3R)-aldose dehydrogenase activity, D-threo-aldose:NAD+ 1-oxidoreductase activity, L-fucose (D-arabinose) dehydrogenase activity, L-fucose dehydrogenase activity, dehydrogenase, L-fucose Relationships: is a type of GO:0016616 Definition: Catalysis of the reaction: a D-threo-aldose + NAD+ = a D-threo-aldono-1,5-lactone + NADH. Sources: EC:1.1.1.122, MetaCyc:D-THREO-ALDOSE-1-DEHYDROGENASE-RXN